positive regulation of axo-dendritic protein transport [GO:1905128] (biological process) Definition: Any process that activates or increases the frequency, rate or extent of axo-dendritic protein transport. References: PMID:20694152 Sources: GOC:TermGenie, GO_REF:0000058 Also known as: up regulation of axo-dendritic protein transport, up-regulation of axo-dendritic protein transport, upregulation of axo-dendritic protein transport, activation of axo-dendritic protein transport, activation of axonal protein transport, positive regulation of axonal protein transport, up regulation of axonal protein transport, up-regulation of axonal protein transport, upregulation of axonal protein transport Relationships: is a type of positive regulation of intracellular protein transport [GO:0090316]; is a type of regulation of axo-dendritic protein transport [GO:1905126]; positively regulates axo-dendritic protein transport [GO:0099640]